{
  "term_id": "UNKNOWN:0001",
  "term_label": "Unknown molecular function",
  "gene": "UniProtKB:O95926",
  "gene_name": "Pre-mRNA-splicing factor SYF2",
  "gene_symbol": "SYF2"
}